{
  "gene_symbol": "KNSTRN",
  "term_id": "GO:0034451",
  "gene_name": "Small kinetochore-associated protein",
  "gene": "UniProtKB:Q9Y448",
  "term_label": "centriolar satellite"
}